{
  "gene_name": "2-Hydroxyacid oxidase 1",
  "gene_symbol": "HAO1",
  "term_id": "UNKNOWN:0003",
  "gene": "UniProtKB:Q9UJM8",
  "term_label": "Unknown cellular component"
}